cholesterol catabolic process [GO:0006707] (biological process) Definition: The chemical reactions and pathways resulting in the breakdown of cholesterol, cholest-5-en-3 beta-ol, the principal sterol of vertebrates and the precursor of many steroids, including bile acids and steroid hormones. Relationships: is_a cholesterol metabolic process [GO:0008203]; is a type of sterol catabolic process [GO:0016127]; is a type of alcohol catabolic process [GO:0046164] Sources: GOC:ai Also known as: cholesterol breakdown, cholesterol catabolism, cholesterol degradation